{
  "gene": "UniProtKB:P24310",
  "gene_symbol": "COX7A1",
  "gene_name": "Cytochrome c oxidase subunit 7A1, mitochondrial",
  "term_id": "GO:0031966",
  "term_label": "mitochondrial membrane"
}